{
  "term_label": "plasma membrane",
  "gene_name": "LIM domain-containing protein 2",
  "gene": "UniProtKB:Q9BT23",
  "term_id": "GO:0005886",
  "gene_symbol": "LIMD2"
}